{
  "term_id": "GO:0005085",
  "gene_symbol": "RINL",
  "gene": "UniProtKB:Q6ZS11",
  "gene_name": "Ras and Rab interactor-like protein",
  "term_label": "guanyl-nucleotide exchange factor activity"
}